{
  "gene_name": "Pro-epidermal growth factor",
  "gene": "UniProtKB:P01133",
  "gene_symbol": "EGF",
  "term_label": "positive regulation of cell population proliferation",
  "term_id": "GO:0008284"
}